{
  "gene_symbol": "TNFAIP2",
  "gene": "UniProtKB:Q03169",
  "term_id": "GO:0006887",
  "term_label": "exocytosis",
  "gene_name": "Tumor necrosis factor alpha-induced protein 2"
}